apoptotic process involved in embryonic digit morphogenesis [GO:1902263] (biological process) Also known as: apoptotic cell death involved in embryonic digit morphogenesis, apoptotic programmed cell death involved in embryonic digit morphogenesis, programmed cell death by apoptosis involved in embryonic digit morphogenesis, apoptosis involved in embryonic digit morphogenesis, apoptotic program involved in embryonic digit morphogenesis, type I programmed cell death involved in embryonic digit morphogenesis, signaling (initiator) caspase activity involved in embryonic digit morphogenesis References: PMID:15967824 Sources: GOC:TermGenie, GOC:dph, GOC:mtg_apoptosis Relationships: is a type of GO:0060561; BFO_0000050 embryonic digit morphogenesis [GO:0042733] Definition: Any apoptotic process that is involved in embryonic digit morphogenesis.